{
  "term_id": "GO:0016323",
  "term_label": "basolateral plasma membrane",
  "gene_symbol": "SLC16A7",
  "gene_name": "Monocarboxylate transporter 2",
  "gene": "UniProtKB:O60669"
}